granzyme B localization to T cell secretory granule [GO:0033380] (biological process) Sources: GOC:mah Relationships: is a type of GO:0033375 Also known as: granzyme B localisation in T cell secretory granule, granzyme B localization in T cell secretory granule, granzyme B localization in T lymphocyte secretory granule, granzyme B localization in T-cell secretory granule, granzyme B localization in T-lymphocyte secretory granule Definition: Any process in which the protease granzyme B is transported to, or maintained in, a location within a secretory granule in a T cell.